{
  "term_id": "UNKNOWN:0002",
  "gene": "UniProtKB:P86480",
  "gene_symbol": "PRR20D",
  "term_label": "Unknown biological process",
  "gene_name": "Proline-rich protein 20D"
}